{
  "gene_symbol": "SCN9A",
  "gene": "UniProtKB:Q15858",
  "term_id": "GO:0086002",
  "gene_name": "Sodium channel protein type 9 subunit alpha",
  "term_label": "cardiac muscle cell action potential involved in contraction"
}